{
  "gene_name": "RISC-loading complex subunit TARBP2",
  "gene_symbol": "TARBP2",
  "term_id": "GO:0030422",
  "term_label": "siRNA processing",
  "gene": "UniProtKB:Q15633"
}